inter-male aggressive behavior [GO:0002121] (biological process) Definition: Aggressive behavior based on competition between males of the same species over access to resources such as females, dominance, status, etc. and characterized by noise, threats, and is often less injurious. Sources: GOC:hjd Also known as: inter-male aggression Relationships: is_a aggressive behavior [GO:0002118]